{
  "gene": "UniProtKB:Q8WWQ2",
  "term_id": "GO:0031012",
  "gene_symbol": "HPSE2",
  "term_label": "extracellular matrix",
  "gene_name": "Inactive heparanase-2"
}